{
  "term_label": "cytoplasmic microtubule organization",
  "gene": "UniProtKB:Q9P2G4",
  "term_id": "GO:0031122",
  "gene_name": "Microtubule-associated protein 10",
  "gene_symbol": "MAP10"
}